{
  "gene": "UniProtKB:Q12756",
  "gene_symbol": "KIF1A",
  "term_id": "GO:0008574",
  "term_label": "plus-end-directed microtubule motor activity",
  "gene_name": "Kinesin-like protein KIF1A"
}